{
  "gene_symbol": "DDX60L",
  "gene_name": "Probable ATP-dependent RNA helicase DDX60-like",
  "gene": "UniProtKB:Q5H9U9",
  "term_id": "GO:0003727",
  "term_label": "single-stranded RNA binding"
}